{
  "term_id": "GO:0003723",
  "gene_name": "Small ribosomal subunit protein eS10",
  "term_label": "RNA binding",
  "gene_symbol": "RPS10",
  "gene": "UniProtKB:P46783"
}